D-ribitol-5-phosphate cytidylyltransferase activity [GO:0047349] (molecular function) Also known as: CTP:D-ribitol-5-phosphate cytidylyltransferase activity, CDP ribitol pyrophosphorylase activity, CDP-ribitol diphosphorylase activity, CDP-ribitol pyrophosphorylase activity, cytidine diphosphate ribitol pyrophosphorylase activity, cytidine diphosphoribitol pyrophosphorylase activity, ribitol 5-phosphate cytidylyltransferase activity Definition: Catalysis of the reaction: D-ribitol 5-phosphate + CTP = CDP-ribitol + diphosphate. Sources: EC:2.7.7.40, RHEA:12456 Relationships: is a type of cytidylyltransferase activity [GO:0070567]